intramolecular oxidoreductase activity, interconverting keto- and enol-groups [GO:0016862] (molecular function) Definition: Catalysis of an oxidation-reduction (redox) reaction in which the hydrogen donor and acceptor, which is a keto- or an enol-group, are the same molecule, and no oxidized product appears. Subtypes: GO:0034018, GO:0043715, GO:0050163, phenylpyruvate tautomerase activity [GO:0050178] Also known as: intramolecular isomerase activity, interconverting keto- and enol-groups Relationships: is a type of intramolecular oxidoreductase activity [GO:0016860] Sources: EC:5.3.2.-, GOC:jl